regulation of cardiac muscle cell membrane repolarization [GO:0099623] (biological process) Subtypes: regulation of ventricular cardiac muscle cell membrane repolarization [GO:0060307], GO:0060372, GO:1905031 Sources: GOC:BHF, GOC:dos, GOC:rl Definition: Any process that modulates the establishment or extent of a change in membrane potential in the polarizing direction towards the resting potential in a cardiomyocyte. Relationships: is a type of GO:0060306; regulates cardiac muscle cell membrane repolarization [GO:0099622] Also known as: regulation of cardiac muscle cell repolarization, regulation of cardiomyocyte membrane repolarization, heart repolarization